ferroptosis [GO:0097707] (BP) Definition: A programmed cell death characterized morphologically by the presence of smaller than normal mitochondria with condensed mitochondrial membrane densities, reduction or vanishing of mitochondria crista, and outer mitochondrial membrane rupture. Activation of mitochondrial voltage-dependent anion channels and mitogen-activated protein kinases, upregulation of endoplasmic reticulum stress, and inhibition of cystine/glutamate antiporter are involved in the induction of ferroptosis. This process is characterized by the accumulation of lipid peroxidation products and lethal reactive oxygen species (ROS) derived from iron metabolism. Glutathione peroxidase 4 (GPX4), heat shock protein beta-1, and nuclear factor erythroid 2-related factor 2 function as negative regulators of ferroptosis by limiting ROS production and reducing cellular iron uptake, respectively. In contrast, NADPH oxidase and p53 act as positive regulators of ferroptosis by promotion of ROS production and inhibition of expression of SLC7A11 (a specific light-chain subunit of the cystine/glutamate antiporter), respectively. Misregulated ferroptosis has been implicated in multiple physiological and pathological processes. Regulation: regulated by regulation of ferroptosis [GO:0110075]; negatively regulated by negative regulation of ferroptosis [GO:0110076]; positively regulated by positive regulation of ferroptosis [GO:0160020] References: PMID:25236395, PMID:26794443 Sources: GOC:mtg_apoptosis Relationships: is a type of programmed cell death [GO:0012501] Also known as: iron-dependent programmed cell death